Cys-tRNA(Pro) deacylase activity [GO:0043907] (molecular function) References: PMID:15886196 Sources: GOC:jl, RHEA:25351 Relationships: is a type of aminoacyl-tRNA deacylase activity [GO:0002161] Also known as: Cys-tRNA(Pro) deacetylase activity, Cys-tRNAPro hydrolase activity Definition: Catalysis of the reaction: L-cysteinyl-tRNA(Pro) + H2O = tRNA(Pro) + L-cysteine + H+.